{
  "gene_symbol": "MAP6",
  "term_label": "dendrite morphogenesis",
  "term_id": "GO:0048813",
  "gene_name": "Microtubule-associated protein 6",
  "gene": "UniProtKB:Q96JE9"
}